{
  "gene_symbol": "DAB2",
  "gene_name": "Disabled homolog 2",
  "gene": "UniProtKB:P98082",
  "term_id": "GO:0010718",
  "term_label": "positive regulation of epithelial to mesenchymal transition"
}